mononeme [GO:0070074] (cellular component) Relationships: is a type of GO:0043231; is part of apical complex [GO:0020007] Definition: A secretory organelle that forms part of the apical complex; a small, threadlike structure located is close proximity to the subpellicular microtubules. Its contents include a rhomboid protease (PfROM1 in Plasmodium falciparum) that moves from the lateral asymmetric localization to the merozoite apical pole and the posterior pole upon release of merozoites from schizonts. References: PMID:18048320 Sources: GOC:BHF